{
  "term_label": "Unknown biological process",
  "term_id": "UNKNOWN:0002",
  "gene_symbol": "IVL",
  "gene_name": "Involucrin",
  "gene": "UniProtKB:P07476"
}